{
  "term_label": "calcium-mediated signaling",
  "gene_symbol": "CX3CR1",
  "gene_name": "CX3C chemokine receptor 1",
  "term_id": "GO:0019722",
  "gene": "UniProtKB:P49238"
}